{
  "gene_name": "Putative uncharacterized protein encoded by LINC00313",
  "term_id": "UNKNOWN:0001",
  "gene_symbol": "LINC00313",
  "gene": "UniProtKB:P59037",
  "term_label": "Unknown molecular function"
}